{
  "term_id": "GO:0031012",
  "gene_name": "CCN family member 1",
  "term_label": "extracellular matrix",
  "gene_symbol": "CCN1",
  "gene": "UniProtKB:O00622"
}